{
  "gene_symbol": "NOTCH2",
  "gene": "UniProtKB:Q04721",
  "gene_name": "Neurogenic locus notch homolog protein 2",
  "term_label": "Unknown molecular function",
  "term_id": "UNKNOWN:0001"
}